{
  "gene_symbol": "CLEC5A",
  "term_label": "Unknown cellular component",
  "term_id": "UNKNOWN:0003",
  "gene_name": "C-type lectin domain family 5 member A",
  "gene": "UniProtKB:Q9NY25"
}